protein deacylation [GO:0035601] (biological process) Subtypes: protein depalmitoylation [GO:0002084], GO:0006476, protein demalonylation [GO:0036046], protein desuccinylation [GO:0036048], GO:0061698, protein depropionylation [GO:0106230], protein depalmitoleylation [GO:1990697] Relationships: is a type of protein modification process [GO:0036211]; is a type of macromolecule deacylation [GO:0098732] References: PMID:12080046 Sources: GOC:se Definition: The removal of an acyl group, any group or radical of the form RCO- where R is an organic group, from a protein amino acid. Also known as: protein amino acid deacylation